{
  "gene_name": "E3 ubiquitin-protein ligase RNF166",
  "term_id": "GO:0061630",
  "term_label": "ubiquitin protein ligase activity",
  "gene_symbol": "RNF166",
  "gene": "UniProtKB:Q96A37"
}